{
  "term_label": "methylglyoxal catabolic process to D-lactate via S-lactoyl-glutathione",
  "gene_symbol": "GATD1",
  "gene": "UniProtKB:Q8NB37",
  "gene_name": "Glutamine amidotransferase-like class 1 domain-containing protein 1",
  "term_id": "GO:0019243"
}